negative regulation of 1-phosphatidyl-1D-myo-inositol 4,5-bisphosphate catabolic process [GO:1902642] (BP) Also known as: down regulation of 1-phosphatidyl-1D-myo-inositol 4,5-bisphosphate breakdown, down regulation of 1-phosphatidyl-1D-myo-inositol 4,5-bisphosphate catabolic process, down regulation of 1-phosphatidyl-1D-myo-inositol 4,5-bisphosphate catabolism, down regulation of 1-phosphatidyl-1D-myo-inositol 4,5-bisphosphate degradation, down-regulation of 1-phosphatidyl-1D-myo-inositol 4,5-bisphosphate breakdown, down-regulation of 1-phosphatidyl-1D-myo-inositol 4,5-bisphosphate catabolic process, down-regulation of 1-phosphatidyl-1D-myo-inositol 4,5-bisphosphate catabolism, down-regulation of 1-phosphatidyl-1D-myo-inositol 4,5-bisphosphate degradation, downregulation of 1-phosphatidyl-1D-myo-inositol 4,5-bisphosphate breakdown, downregulation of 1-phosphatidyl-1D-myo-inositol 4,5-bisphosphate catabolic process, downregulation of 1-phosphatidyl-1D-myo-inositol 4,5-bisphosphate catabolism, downregulation of 1-phosphatidyl-1D-myo-inositol 4,5-bisphosphate degradation, negative regulation of 1-phosphatidyl-1D-myo-inositol 4,5-bisphosphate breakdown, negative regulation of 1-phosphatidyl-1D-myo-inositol 4,5-bisphosphate catabolism, negative regulation of 1-phosphatidyl-1D-myo-inositol 4,5-bisphosphate degradation, inhibition of 1-phosphatidyl-1D-myo-inositol 4,5-bisphosphate breakdown, inhibition of 1-phosphatidyl-1D-myo-inositol 4,5-bisphosphate catabolic process, inhibition of 1-phosphatidyl-1D-myo-inositol 4,5-bisphosphate catabolism, inhibition of 1-phosphatidyl-1D-myo-inositol 4,5-bisphosphate degradation Definition: Any process that stops, prevents or reduces the frequency, rate or extent of 1-phosphatidyl-1D-myo-inositol 4,5-bisphosphate catabolic process. Relationships: is a type of negative regulation of lipid catabolic process [GO:0050995]; is a type of regulation of 1-phosphatidyl-1D-myo-inositol 4,5-bisphosphate catabolic process [GO:1902641]; is a type of negative regulation of phospholipid metabolic process [GO:1903726]; negatively regulates GO:1902634 References: PMID:22562153 Sources: GOC:TermGenie, GOC:di, GO_REF:0000058